{
  "term_label": "regulation of immune system process",
  "gene": "UniProtKB:Q96K62",
  "gene_name": "Zinc finger and BTB domain-containing protein 45",
  "term_id": "GO:0002682",
  "gene_symbol": "ZBTB45"
}